organic acid phosphorylation [GO:0031388] (biological process) Sources: GOC:mah Definition: The process of introducing one or more phosphate groups into an organic acid. Relationships: is a type of organic acid metabolic process [GO:0006082]; is a type of phosphorylation [GO:0016310]